{
  "gene_symbol": "ZNHIT3",
  "gene": "UniProtKB:Q15649",
  "gene_name": "Zinc finger HIT domain-containing protein 3",
  "term_id": "UNKNOWN:0001",
  "term_label": "Unknown molecular function"
}